low-affinity D-glucose:sodium symporter activity [GO:0005362] (MF) Definition: Enables the transfer of a solute or solutes from one side of a membrane to the other according to the reaction: D-glucose(out) + Na+(out) = D-glucose(in) + Na+(in). In low-affinity transport the transporter is able to bind the solute only if it is present at very high concentrations. Sources: TC:2.A.21.3.- Also known as: low-affinity glucose-sodium cotransporter activity, low-affinity glucose:sodium symporter activity Relationships: is_a D-glucose:sodium symporter activity [GO:0005412]